{
  "term_id": "GO:0016407",
  "term_label": "acetyltransferase activity",
  "gene": "UniProtKB:Q00403",
  "gene_symbol": "GTF2B",
  "gene_name": "Transcription initiation factor IIB"
}